{
  "gene_name": "Thymosin beta 15B",
  "term_id": "UNKNOWN:0003",
  "gene": "UniProtKB:A0A087X1C1",
  "gene_symbol": "TMSB15B",
  "term_label": "Unknown cellular component"
}